{
  "gene": "UniProtKB:Q9H305",
  "gene_name": "Cell death-inducing p53-target protein 1",
  "gene_symbol": "CDIP1",
  "term_label": "cytoplasmic side of lysosomal membrane",
  "term_id": "GO:0098574"
}